{
  "gene_name": "Stress-70 protein, mitochondrial",
  "gene": "UniProtKB:P38646",
  "gene_symbol": "HSPA9",
  "term_label": "protein refolding",
  "term_id": "GO:0042026"
}